{
  "gene_name": "Thrombopoietin",
  "term_label": "thrombopoietin-mediated signaling pathway",
  "gene": "UniProtKB:P40225",
  "gene_symbol": "THPO",
  "term_id": "GO:0038163"
}